{
  "gene_symbol": "NPHP4",
  "term_id": "UNKNOWN:0001",
  "gene": "UniProtKB:O75161",
  "term_label": "Unknown molecular function",
  "gene_name": "Nephrocystin-4"
}